negative regulation of actin cortical patch assembly [GO:0120133] (biological process) References: PMID:19962315 Definition: Any process that stops, prevents, or reduces the frequency, rate or extent of the assembly of actin cortical patches. Also known as: down regulation of actin cortical patch assembly, down-regulation of actin cortical patch assembly, downregulation of actin cortical patch assembly, inhibition of actin cortical patch assembly Relationships: is_a regulation of actin cytoskeleton organization [GO:0032956]; is a type of regulation of cellular component biogenesis [GO:0044087]; is a type of negative regulation of cytoskeleton organization [GO:0051494]; negatively regulates GO:0000147